{
  "gene_symbol": "EPHA4",
  "term_label": "transmembrane-ephrin receptor activity",
  "term_id": "GO:0005005",
  "gene": "UniProtKB:P54764",
  "gene_name": "Ephrin type-A receptor 4"
}